{
  "gene_symbol": "VPS26B",
  "gene": "UniProtKB:Q4G0F5",
  "term_label": "endosome",
  "term_id": "GO:0005768",
  "gene_name": "Vacuolar protein sorting-associated protein 26B"
}